{
  "term_id": "GO:0008009",
  "gene": "UniProtKB:P10147",
  "term_label": "chemokine activity",
  "gene_name": "C-C motif chemokine 3",
  "gene_symbol": "CCL3"
}